{
  "term_label": "regulation of vascular endothelial growth factor receptor signaling pathway",
  "term_id": "GO:0030947",
  "gene_symbol": "TMEM204",
  "gene": "UniProtKB:Q9BSN7",
  "gene_name": "Transmembrane protein 204"
}